{
  "gene_name": "Uncharacterized protein C17orf113",
  "term_label": "Unknown cellular component",
  "gene": "UniProtKB:A0A1B0GUU1",
  "term_id": "UNKNOWN:0003",
  "gene_symbol": "C17orf113"
}